{
  "gene_name": "Adenomatous polyposis coli protein 2",
  "gene": "UniProtKB:O95996",
  "term_label": "negative regulation of microtubule depolymerization",
  "gene_symbol": "APC2",
  "term_id": "GO:0007026"
}